{
  "gene": "UniProtKB:Q12983",
  "term_id": "GO:0043068",
  "gene_symbol": "BNIP3",
  "term_label": "positive regulation of programmed cell death",
  "gene_name": "BCL2_adenovirus E1B 19 kDa protein-interacting protein 3"
}